{
  "term_label": "nucleolus",
  "term_id": "GO:0005730",
  "gene_name": "Probable ribosome biogenesis protein RLP24",
  "gene_symbol": "RSL24D1",
  "gene": "UniProtKB:Q9UHA3"
}